{
  "gene_symbol": "TPT1",
  "gene": "UniProtKB:P13693",
  "term_label": "Unknown biological process",
  "term_id": "UNKNOWN:0002",
  "gene_name": "Translationally-controlled tumor protein"
}